{
  "gene_name": "Caspase-7",
  "gene": "UniProtKB:P55210",
  "gene_symbol": "CASP7",
  "term_label": "cytoplasm",
  "term_id": "GO:0005737"
}